intermicrovillar adhesion [GO:0090675] (BP) Definition: The cell-cell adhesion process by which adjacent microvilli attach to each other through Ca(2+)-dependent adhesion links made of protocadherin-24 and mucin-like protocadherin. References: PMID:24725409 Sources: GOC:lb Relationships: is a type of homotypic cell-cell adhesion [GO:0034109]; is part of GO:1904970